oxidoreductase activity, acting on the CH-NH2 group of donors, iron-sulfur protein as acceptor [GO:0016643] (MF) Definition: Catalysis of an oxidation-reduction (redox) reaction in which a CH-NH2 group acts as a hydrogen or electron donor and reduces an iron-sulfur protein. Subtypes: glutamate synthase (ferredoxin) activity [GO:0016041] Also known as: oxidoreductase activity, acting on the CH-NH2 group of donors, iron-sulphur protein as acceptor Relationships: is a type of GO:0016638 Sources: GOC:ai